interleukin-19 receptor activity [GO:0042014] (molecular function) Sources: GOC:jl, GOC:signaling Relationships: is a type of cytokine receptor activity [GO:0004896]; has part interleukin-19 binding [GO:0042013] Definition: Combining with interleukin-19 and transmitting the signal from one side of the membrane to the other to initiate a change in cell activity. Also known as: IL-19 receptor activity, IL-19R